{
  "gene_name": "5-aminolevulinate synthase, non-specific, mitochondrial",
  "term_label": "hemoglobin biosynthetic process",
  "gene_symbol": "ALAS1",
  "gene": "UniProtKB:P13196",
  "term_id": "GO:0042541"
}